negative regulation of early endosome to late endosome transport [GO:2000642] (BP) Relationships: is a type of GO:0032387; is a type of regulation of early endosome to late endosome transport [GO:2000641]; negatively regulates GO:0045022 Definition: Any process that stops, prevents or reduces the frequency, rate or extent of early endosome to late endosome transport. Sources: GOC:BHF